detection of muscle activity [GO:0014864] (biological process) Relationships: is_a response to muscle activity [GO:0014850]; is a type of GO:0014865 Subtypes: GO:0014875 Definition: The series of events in which a muscle activity stimulus is received by a cell and converted into a molecular signal. Sources: GOC:mtg_muscle